{
  "gene": "UniProtKB:P00395",
  "gene_symbol": "MT-CO1",
  "term_label": "respiratory electron transport chain",
  "term_id": "GO:0022904",
  "gene_name": "Cytochrome c oxidase subunit 1"
}